{
  "gene_name": "Myeloma-overexpressed gene protein",
  "gene": "UniProtKB:Q96EZ4",
  "term_id": "UNKNOWN:0002",
  "gene_symbol": "MYEOV",
  "term_label": "Unknown biological process"
}